{
  "gene_name": "Golgin subfamily A member 8H",
  "gene": "UniProtKB:P0CJ92",
  "term_label": "Golgi cis cisterna",
  "term_id": "GO:0000137",
  "gene_symbol": "GOLGA8H"
}